{
  "gene_name": "CDK5 regulatory subunit-associated protein 2",
  "term_id": "GO:0090266",
  "term_label": "regulation of mitotic cell cycle spindle assembly checkpoint",
  "gene_symbol": "CDK5RAP2",
  "gene": "UniProtKB:Q96SN8"
}